{
  "gene_symbol": "OR2B8",
  "gene_name": "Putative olfactory receptor 2B8",
  "term_id": "GO:0005886",
  "gene": "UniProtKB:P59922",
  "term_label": "plasma membrane"
}